{
  "term_label": "actinin binding",
  "gene": "UniProtKB:P50461",
  "gene_symbol": "CSRP3",
  "term_id": "GO:0042805",
  "gene_name": "Cysteine and glycine-rich protein 3"
}